{
  "gene_name": "Cytochrome P450 2A7",
  "term_id": "GO:0020037",
  "gene": "UniProtKB:P20853",
  "gene_symbol": "CYP2A7",
  "term_label": "heme binding"
}